{
  "gene_name": "Double homeobox protein B",
  "term_id": "GO:0006357",
  "gene": "UniProtKB:A0A1W2PPF3",
  "gene_symbol": "DUXB",
  "term_label": "regulation of transcription by RNA polymerase II"
}